{
  "gene": "UniProtKB:Q6H3X3",
  "gene_name": "UL-16 binding protein 5",
  "term_label": "external side of plasma membrane",
  "term_id": "GO:0009897",
  "gene_symbol": "RAET1G"
}